{
  "gene": "UniProtKB:P51654",
  "term_label": "cell surface",
  "term_id": "GO:0009986",
  "gene_name": "Glypican-3",
  "gene_symbol": "GPC3"
}